{
  "gene": "UniProtKB:Q7Z6P3",
  "term_id": "UNKNOWN:0003",
  "term_label": "Unknown cellular component",
  "gene_symbol": "RAB44",
  "gene_name": "Ras-related protein Rab-44"
}